{
  "term_label": "serine-tRNA ligase activity",
  "gene_symbol": "SARS1",
  "gene": "UniProtKB:P49591",
  "gene_name": "Serine--tRNA ligase, cytoplasmic",
  "term_id": "GO:0004828"
}